{
  "gene_symbol": "KRTAP9-4",
  "gene_name": "Keratin-associated protein 9-4",
  "gene": "UniProtKB:Q9BYQ2",
  "term_label": "Unknown molecular function",
  "term_id": "UNKNOWN:0001"
}